{
  "gene_symbol": "GYPC",
  "gene": "UniProtKB:P04921",
  "term_id": "GO:0030863",
  "gene_name": "Glycophorin-C",
  "term_label": "cortical cytoskeleton"
}